{
  "term_label": "Unknown cellular component",
  "term_id": "UNKNOWN:0003",
  "gene_symbol": "RPP38-DT",
  "gene": "UniProtKB:Q8N326",
  "gene_name": "Putative uncharacterized protein RPP38-DT"
}